bronchus cartilage morphogenesis [GO:0060533] (biological process) Relationships: is a type of cartilage morphogenesis [GO:0060536]; is part of bronchus morphogenesis [GO:0060434]; is part of bronchus cartilage development [GO:0060532] Sources: GOC:dph Definition: The process in which the bronchus cartilage is generated and organized. The bronchus cartilage is the connective tissue of the portion of the airway that connects to the lungs.